{
  "gene_name": "Olfactory receptor 8U9",
  "term_label": "Unknown molecular function",
  "gene_symbol": "OR8U9",
  "term_id": "UNKNOWN:0001",
  "gene": "UniProtKB:P0C7N5"
}